G protein-coupled acetylcholine receptor binding [GO:0031789] (molecular function) Definition: Binding to a G protein-coupled acetylcholine receptor. Sources: GOC:bf, GOC:mah, GOC:nln Also known as: G-protein coupled acetylcholine receptor binding, muscarinic acetylcholine receptor binding, M1 muscarinic acetylcholine receptor binding, M1 muscarinic acetylcholine receptor ligand, M2 muscarinic acetylcholine receptor binding, M2 muscarinic acetylcholine receptor ligand, M3 muscarinic acetylcholine receptor binding, M3 muscarinic acetylcholine receptor ligand, M4 muscarinic acetylcholine receptor binding, M4 muscarinic acetylcholine receptor ligand, M5 muscarinic acetylcholine receptor binding, M5 muscarinic acetylcholine receptor ligand, muscarinic acetylcholine receptor ligand Relationships: is a type of GO:0001664